detection of temperature stimulus [GO:0016048] (biological process) Definition: The series of events in which a temperature stimulus (hot or cold) is received and converted into a molecular signal. Sources: GOC:hb Also known as: detection of temperature, detection of thermal stimulus, perception of temperature Relationships: is a type of response to temperature stimulus [GO:0009266]; is_a detection of external stimulus [GO:0009581]; is a type of GO:0009582 Subtypes: detection of temperature stimulus involved in sensory perception [GO:0050961]